{
  "gene": "UniProtKB:Q9BX67",
  "term_id": "GO:0098609",
  "gene_name": "Junctional adhesion molecule C",
  "gene_symbol": "JAM3",
  "term_label": "cell-cell adhesion"
}